{
  "gene_symbol": "TRPV3",
  "term_label": "calcium ion import across plasma membrane",
  "gene_name": "Transient receptor potential cation channel subfamily V member 3",
  "term_id": "GO:0098703",
  "gene": "UniProtKB:Q8NET8"
}